antimicrobial humoral immune response mediated by antimicrobial peptide [GO:0061844] (biological process) Relationships: is a type of antimicrobial humoral response [GO:0019730] Definition: An immune response against microbes mediated by anti-microbial peptides in body fluid. Also known as: peptide-mediated antimicrobial humoral response, antimicrobial peptide-mediated antimicrobial humoral response References: PMID:15761415, PMID:24287494